{
  "term_id": "UNKNOWN:0002",
  "term_label": "Unknown biological process",
  "gene_symbol": "A0A6Q8PGS0",
  "gene": "UniProtKB:A0A6Q8PGS0",
  "gene_name": "Uncharacterized protein"
}